{
  "term_label": "negative regulation of Wnt signaling pathway",
  "term_id": "GO:0030178",
  "gene_symbol": "NKD2",
  "gene": "UniProtKB:Q969F2",
  "gene_name": "Protein naked cuticle homolog 2"
}